{
  "gene_symbol": "GHITM",
  "term_id": "GO:0099093",
  "gene": "UniProtKB:Q9H3K2",
  "gene_name": "Growth hormone-inducible transmembrane protein",
  "term_label": "calcium export from the mitochondrion"
}